{
  "gene_name": "Trafficking protein particle complex subunit 6A",
  "term_id": "GO:0005801",
  "term_label": "cis-Golgi network",
  "gene_symbol": "TRAPPC6A",
  "gene": "UniProtKB:O75865"
}